{
  "term_id": "GO:0006364",
  "term_label": "rRNA processing",
  "gene_name": "Proline-, glutamic acid- and leucine-rich protein 1",
  "gene": "UniProtKB:Q8IZL8",
  "gene_symbol": "PELP1"
}